{
  "term_id": "GO:0036126",
  "gene_symbol": "TCP11X1",
  "gene_name": "T-complex protein 11 X-linked protein 1",
  "term_label": "sperm flagellum",
  "gene": "UniProtKB:B4DZS4"
}